regulation of systemic arterial blood pressure by endothelin [GO:0003100] (biological process) Sources: GOC:mtg_cardio Definition: The process in which endothelin modulates the force with which blood passes through the circulatory system. Endothelin is a hormone that is released by the endothelium, and it is a vasoconstrictor. Relationships: is a type of regulation of systemic arterial blood pressure by hormone [GO:0001990]